{
  "gene_name": "Chromosome alignment-maintaining phosphoprotein 1",
  "gene": "UniProtKB:Q96JM3",
  "term_label": "protein localization to microtubule",
  "term_id": "GO:0035372",
  "gene_symbol": "CHAMP1"
}